{
  "gene_name": "Golgi apparatus protein 1",
  "term_id": "GO:0000139",
  "gene_symbol": "GLG1",
  "gene": "UniProtKB:Q92896",
  "term_label": "Golgi membrane"
}